{
  "term_label": "Unknown molecular function",
  "term_id": "UNKNOWN:0001",
  "gene_name": "Attractin",
  "gene_symbol": "ATRN",
  "gene": "UniProtKB:O75882"
}